amyloid-beta clearance by cellular catabolic process [GO:0150094] (biological process) References: PMID:18289866 Sources: GOC:aruk, GOC:bc Definition: The process in which amyloid-beta is removed from extracellular brain regions by cell surface receptor-mediated endocytosis, followed by intracellular degradation. Relationships: is a type of GO:0009056; is a type of amyloid-beta metabolic process [GO:0050435]; is a type of amyloid-beta clearance [GO:0097242] Also known as: amyloid-beta clearance by phagocytosis